{
  "gene_name": "Cytochrome P450 4A22",
  "gene_symbol": "CYP4A22",
  "gene": "UniProtKB:Q5TCH4",
  "term_id": "GO:0043651",
  "term_label": "linoleic acid metabolic process"
}